{
  "term_id": "GO:0015914",
  "term_label": "phospholipid transport",
  "gene_symbol": "TNFAIP8L3",
  "gene": "UniProtKB:Q5GJ75",
  "gene_name": "Tumor necrosis factor alpha-induced protein 8-like protein 3"
}